{
  "gene": "UniProtKB:Q30KQ5",
  "gene_name": "Beta-defensin 115",
  "gene_symbol": "DEFB115",
  "term_label": "innate immune response",
  "term_id": "GO:0045087"
}